protein localization to chromosome [GO:0034502] (BP) Relationships: is a type of protein localization to organelle [GO:0033365] Subtypes: GO:0034503, GO:0070198, protein localization to chromatin [GO:0071168], GO:0071459, protein localization to condensed chromosome [GO:1903083], protein localization to site of double-strand break [GO:1990166] Definition: Any process in which a protein is transported to, or maintained at, a specific location on a chromosome. Also known as: protein localisation to chromosome, condensin localization to chromosome Sources: GOC:mah